{
  "gene_symbol": "GOLGA6L22",
  "gene_name": "Golgin subfamily A member 6-like protein 22",
  "term_id": "UNKNOWN:0001",
  "gene": "UniProtKB:H0YM25",
  "term_label": "Unknown molecular function"
}